{
  "gene": "UniProtKB:Q08830",
  "gene_name": "Fibrinogen-like protein 1",
  "gene_symbol": "FGL1",
  "term_label": "negative regulation of T cell activation",
  "term_id": "GO:0050868"
}